regulation of SREBP signaling pathway [GO:2000638] (biological process) Also known as: regulation of SREBP-mediated signaling pathway, regulation of SREBP-mediated signalling pathway Definition: Any process that modulates the frequency, rate or extent of the SREBP signaling pathway. Relationships: is a type of regulation of cellular response to stress [GO:0080135]; is a type of regulation of intracellular signal transduction [GO:1902531]; regulates SREBP signaling pathway [GO:0032933] Subtypes: GO:2000639, GO:2000640 Sources: GOC:BHF